{
  "term_id": "GO:0019948",
  "gene_name": "SUMO-activating enzyme subunit 2",
  "gene": "UniProtKB:Q9UBT2",
  "term_label": "SUMO activating enzyme activity",
  "gene_symbol": "UBA2"
}